cadmium ion import into vacuole [GO:0036249] (biological process) Relationships: is a type of vacuolar transmembrane transport [GO:0034486]; is a type of cadmium ion transmembrane transport [GO:0070574] Also known as: vacuolar cadmium import Definition: The directed movement of cadmium ions into the vacuole. Sources: GOC:al